{
  "term_label": "Unknown cellular component",
  "gene_symbol": "SDR9C7",
  "gene": "UniProtKB:Q8NEX9",
  "gene_name": "Short-chain dehydrogenase_reductase family 9C member 7",
  "term_id": "UNKNOWN:0003"
}